{
  "term_label": "ciliary basal body",
  "gene": "UniProtKB:Q494V2",
  "gene_name": "Cilia- and flagella-associated protein 100",
  "gene_symbol": "CFAP100",
  "term_id": "GO:0036064"
}